{
  "term_label": "Unknown cellular component",
  "gene_symbol": "OR14L1",
  "gene": "UniProtKB:Q8NHC6",
  "gene_name": "Olfactory receptor 14L1",
  "term_id": "UNKNOWN:0003"
}